{
  "term_id": "GO:0007165",
  "gene_symbol": "IMPA2",
  "gene_name": "Inositol monophosphatase 2",
  "gene": "UniProtKB:O14732",
  "term_label": "signal transduction"
}